aminophospholipid translocation [GO:0140331] (BP) Definition: The movement of an aminophospholipid molecule from one leaflet of a membrane bilayer to the opposite leaflet. Sources: GOC:pg Relationships: is a type of aminophospholipid transport [GO:0015917]; is a type of phospholipid translocation [GO:0045332]